tocopherol C-methyltransferase activity [GO:0050342] (molecular function) Also known as: gamma-tocopherol methyltransferase activity, tocopherol O-methyltransferase activity, S-adenosyl-L-methionine:gamma-tocopherol 5-O-methyltransferase activity Sources: EC:2.1.1.95 Definition: Catalysis of the reaction: gamma-tocopherol + S-adenosyl-L-methionine = (+)-alpha-tocopherol + H+ + S-adenosyl-L-homocysteine. This reaction can also use delta-tocopherol, gamma-tocotrienol and delta-tocotrienol as substrates. Relationships: is a type of O-methyltransferase activity [GO:0008171]